{
  "gene": "UniProtKB:P09972",
  "term_label": "glycolytic process",
  "term_id": "GO:0006096",
  "gene_name": "Fructose-bisphosphate aldolase C",
  "gene_symbol": "ALDOC"
}